monocyte extravasation [GO:0035696] (biological process) References: PMID:10657654 Sources: CL:0000576, GOC:BHF Relationships: is a type of cellular extravasation [GO:0045123]; is a type of mononuclear cell migration [GO:0071674]; is a type of myeloid leukocyte migration [GO:0097529] Regulation: regulated by regulation of monocyte extravasation [GO:2000437]; negatively regulated by negative regulation of monocyte extravasation [GO:2000438]; positively regulated by positive regulation of monocyte extravasation [GO:2000439] Definition: The migration of a monocyte from the blood vessels into the surrounding tissue.